{
  "term_id": "UNKNOWN:0001",
  "gene_name": "Zinc transporter ZIP9",
  "term_label": "Unknown molecular function",
  "gene_symbol": "SLC39A9",
  "gene": "UniProtKB:Q9NUM3"
}